{
  "gene_symbol": "ZPBP",
  "term_label": "binding of sperm to zona pellucida",
  "term_id": "GO:0007339",
  "gene_name": "Zona pellucida-binding protein 1",
  "gene": "UniProtKB:Q9BS86"
}